regulation of endocrocin biosynthetic process [GO:1900667] (biological process) Relationships: is a type of regulation of ketone biosynthetic process [GO:0010566]; is a type of regulation of secondary metabolite biosynthetic process [GO:1900376]; regulates endocrocin biosynthetic process [GO:1900602] Definition: Any process that modulates the frequency, rate or extent of endocrocin biosynthetic process. Also known as: regulation of endocrocin anabolism, regulation of endocrocin biosynthesis, regulation of endocrocin formation, regulation of endocrocin synthesis Subtypes: GO:1900668, positive regulation of endocrocin biosynthetic process [GO:1900669] Sources: GOC:TermGenie, GOC:di